regulation of calcineurin-NFAT signaling cascade [GO:0070884] (biological process) Definition: Any process that modulates the frequency, rate or extent of the calcineurin-NFAT signaling cascade. Sources: GOC:ai Also known as: regulation of calcineurin-NFAT signalling cascade, NFAT protein import into nucleus, regulation of NFAT protein import into nucleus, regulation of calcineurin-NFAT signaling pathway Subtypes: GO:0070885, positive regulation of calcineurin-NFAT signaling cascade [GO:0070886] Relationships: is a type of regulation of calcineurin-mediated signaling [GO:0106056]; RO_0002211 calcineurin-NFAT signaling cascade [GO:0033173]